Roundabout binding [GO:0048495] (molecular function) Definition: Binding to Roundabout (ROBO) receptor, a transmembrane receptor. References: PMID:10102268, PMID:10197527 Sources: GOC:ecd Also known as: Roundabout receptor binding Relationships: is a type of signaling receptor binding [GO:0005102]